{
  "term_label": "actin filament binding",
  "gene": "UniProtKB:Q8N3F8",
  "gene_name": "MICAL-like protein 1",
  "term_id": "GO:0051015",
  "gene_symbol": "MICALL1"
}